{
  "term_label": "Unknown molecular function",
  "gene_symbol": "HRES1",
  "term_id": "UNKNOWN:0001",
  "gene": "UniProtKB:P13985",
  "gene_name": "Putative HTLV-1-related endogenous sequence"
}